SAGA-type complex [GO:0070461] (cellular component) Subtypes: SAGA complex [GO:0000124], transcription factor TFTC complex [GO:0033276], SLIK (SAGA-like) complex [GO:0046695], ADA complex [GO:0140671], ATAC complex [GO:0140672] Also known as: SAGA family complex Definition: A histone acetyltransferase complex that acetylates nucleosomal histones H2B, H3, or H4 and is required for the expression of a subset of Pol II-transcribed genes. This complex includes the acetyltransferases GCN5/KAT2A or PCAF/KAT2B, several proteins of the ADA, SGF and SPT families, and several TBP-associate proteins (TAFs). Relationships: is a type of histone acetyltransferase complex [GO:0000123] References: PMID:10637607, PMID:17337012 Sources: GOC:mah